{
  "term_id": "GO:0016300",
  "gene": "UniProtKB:Q8IYL2",
  "gene_name": "Probable tRNA (uracil-O(2)-)-methyltransferase",
  "term_label": "tRNA (uridine) methyltransferase activity",
  "gene_symbol": "TRMT44"
}